{
  "term_label": "extracellular matrix",
  "gene_symbol": "TIMP2",
  "gene_name": "Metalloproteinase inhibitor 2",
  "gene": "UniProtKB:P16035",
  "term_id": "GO:0031012"
}